fibrillar center [GO:0001650] (cellular component) Also known as: fibrillar centre Relationships: is a type of cellular anatomical structure [GO:0110165]; is part of nucleolus [GO:0005730] Definition: A structure found most metazoan nucleoli, but not usually found in lower eukaryotes; surrounded by the dense fibrillar component; the zone of transcription from multiple copies of the pre-rRNA genes is in the border region between these two structures. References: PMID:10754561